{
  "gene": "UniProtKB:Q8N8E2",
  "term_id": "GO:0006355",
  "gene_symbol": "ZNF513",
  "gene_name": "Zinc finger protein 513",
  "term_label": "regulation of DNA-templated transcription"
}